{
  "gene_name": "Galectin-9B",
  "gene_symbol": "LGALS9B",
  "term_id": "GO:0016936",
  "gene": "UniProtKB:Q3B8N2",
  "term_label": "galactoside binding"
}